{
  "gene_symbol": "ADGRL4",
  "term_id": "GO:0007186",
  "gene_name": "Adhesion G protein-coupled receptor L4",
  "term_label": "G protein-coupled receptor signaling pathway",
  "gene": "UniProtKB:Q9HBW9"
}